{
  "term_id": "GO:0050778",
  "term_label": "positive regulation of immune response",
  "gene_symbol": "HLA-DPA1",
  "gene": "UniProtKB:P20036",
  "gene_name": "HLA class II histocompatibility antigen, DP alpha 1 chain"
}